thermospermine oxidase activity [GO:1990534] (molecular function) Definition: Catalysis of the reaction: S-methyl-5'-thioadenosine + thermospermine + H+ = S-adenosyl 3-(methylthio)propylamine + spermidine. References: PMID:24906355 Sources: RHEA:57836 Relationships: is a type of GO:0046592